positive regulation of chlorophyll catabolic process [GO:1903648] (biological process) Also known as: positive regulation of chlorophyll breakdown, positive regulation of chlorophyll catabolism, positive regulation of chlorophyll degradation, up regulation of chlorophyll breakdown, up regulation of chlorophyll catabolic process, up regulation of chlorophyll catabolism, up regulation of chlorophyll degradation, up-regulation of chlorophyll breakdown, up-regulation of chlorophyll catabolic process, up-regulation of chlorophyll catabolism, up-regulation of chlorophyll degradation, upregulation of chlorophyll breakdown, upregulation of chlorophyll catabolic process, upregulation of chlorophyll catabolism, upregulation of chlorophyll degradation, activation of chlorophyll breakdown, activation of chlorophyll catabolic process, activation of chlorophyll catabolism, activation of chlorophyll degradation Relationships: is a type of regulation of chlorophyll catabolic process [GO:0010271]; is a type of positive regulation of tetrapyrrole catabolic process [GO:1901406]; positively regulates chlorophyll catabolic process [GO:0015996] Definition: Any process that activates or increases the frequency, rate or extent of chlorophyll catabolic process. References: PMID:24719469 Sources: GOC:TermGenie, GO_REF:0000058